L-alanine catabolic process [GO:0042853] (biological process) Sources: GOC:jl, GOC:jsg, GOC:mah Also known as: L-alanine breakdown, L-alanine catabolism, L-alanine degradation Definition: The chemical reactions and pathways resulting in the breakdown of L-alanine, the L-enantiomer of 2-aminopropanoic acid, i.e. (2S)-2-aminopropanoic acid. Subtypes: L-alanine oxidation to D-lactate and ammonia [GO:0019479], L-alanine oxidation to pyruvate via D-alanine [GO:0019480], L-alanine catabolic process, by transamination [GO:0019481], GO:0019667 Relationships: is a type of alanine catabolic process [GO:0006524]; is a type of GO:0042851; is a type of GO:0170035; is a type of GO:0170040